{
  "gene_name": "Serine_arginine-rich splicing factor 1",
  "term_id": "GO:0000381",
  "gene": "UniProtKB:Q07955",
  "gene_symbol": "SRSF1",
  "term_label": "regulation of alternative mRNA splicing, via spliceosome"
}